{
  "gene_symbol": "GABRG3",
  "term_label": "GABA-A receptor activity",
  "term_id": "GO:0004890",
  "gene_name": "Gamma-aminobutyric acid receptor subunit gamma-3",
  "gene": "UniProtKB:Q99928"
}